{
  "gene_symbol": "ZNF625",
  "gene_name": "Zinc finger protein 625",
  "gene": "UniProtKB:Q96I27",
  "term_id": "GO:0006357",
  "term_label": "regulation of transcription by RNA polymerase II"
}